protein methylation [GO:0006479] (biological process) Sources: GOC:ai Relationships: is a type of GO:0008213; is a type of macromolecule methylation [GO:0043414] Definition: The addition of a methyl group to a protein amino acid. A methyl group is derived from methane by the removal of a hydrogen atom. Subtypes: GO:0006480, C-terminal protein methylation [GO:0006481], peptidyl-histidine methylation [GO:0018021], peptidyl-lysine methylation [GO:0018022], peptidyl-cysteine methylation [GO:0018125], peptidyl-arginine methylation [GO:0018216], GO:0018364 Also known as: protein amino acid methylation